{
  "gene_symbol": "RAD23A",
  "term_id": "GO:0043130",
  "term_label": "ubiquitin binding",
  "gene_name": "UV excision repair protein RAD23 homolog A",
  "gene": "UniProtKB:P54725"
}